{
  "gene_symbol": "TBX15",
  "gene": "UniProtKB:Q96SF7",
  "term_label": "RNA polymerase II cis-regulatory region sequence-specific DNA binding",
  "term_id": "GO:0000978",
  "gene_name": "T-box transcription factor TBX15"
}